sporangium germination [GO:0075222] (biological process) Also known as: germination of symbiont sporangium on or near host, sporangium germination on or near host, symbiont sporangium germination on or near host, direct germination on or near host Relationships: is a type of sporangium development [GO:0043582] Regulation: regulated by regulation of sporangium germination [GO:0075223]; positively regulated by GO:0075224; negatively regulated by GO:0075225 Sources: GOC:pamgo_curators Definition: The physiological, developmental and morphological changes that occur in a symbiont sporangium following release from dormancy up to the earliest signs of growth. A sporangium is a structure producing and containing spores.